{
  "gene_name": "Interleukin-1 family member 10",
  "gene": "UniProtKB:Q8WWZ1",
  "term_label": "extracellular space",
  "gene_symbol": "IL1F10",
  "term_id": "GO:0005615"
}